{
  "term_id": "GO:0005737",
  "term_label": "cytoplasm",
  "gene_symbol": "ARHGEF11",
  "gene_name": "Rho guanine nucleotide exchange factor 11",
  "gene": "UniProtKB:O15085"
}